cellular response to diphenidol [GO:1904561] (biological process) References: PMID:25796330 Sources: GOC:TermGenie, GOC:mr, GO_REF:0000071 Relationships: is a type of cellular response to alcohol [GO:0097306]; is a type of cellular response to nitrogen compound [GO:1901699]; is a type of GO:1904560 Definition: Any process that results in a change in state or activity of a cell (in terms of movement, secretion, enzyme production, gene expression, etc.) as a result of a diphenidol stimulus.